{
  "gene_name": "Serine_threonine-protein kinase ICK",
  "gene": "UniProtKB:Q9UPZ9",
  "gene_symbol": "CILK1",
  "term_id": "GO:0004674",
  "term_label": "protein serine/threonine kinase activity"
}